pore-forming activity [GO:0140911] (molecular function) Definition: An activity in which a protein is inserted into the membrane of another cell where it forms transmembrane pores. Pores disrupts the integrity of the cell membrane, resulting in deregulated ion homeostasis, cellular dysfunction, and can result in cell death. References: PMID:1406491, PMID:25157079, PMID:34387717 Also known as: pore forming activity, canonical holin activity, holin activity, pinholin activity Relationships: is a type of molecular_function [GO:0003674]